response to antipsychotic drug [GO:0097332] (biological process) Relationships: is a type of response to chemical [GO:0042221] Sources: GOC:pr Definition: Any process that results in a change in state or activity of a cell or an organism (in terms of movement, secretion, enzyme production, gene expression, etc.) as a result of an antipsychotic drug stimulus. Antipsychotic drugs are agents that control agitated psychotic behaviour, alleviate acute psychotic states, reduce psychotic symptoms, and exert a quieting effect.